{
  "term_id": "GO:0000976",
  "gene": "UniProtKB:P29374",
  "gene_symbol": "ARID4A",
  "gene_name": "AT-rich interactive domain-containing protein 4A",
  "term_label": "transcription cis-regulatory region binding"
}